{
  "gene_name": "Serine_threonine_tyrosine-interacting-like protein 2",
  "term_label": "protein tyrosine/serine/threonine phosphatase activity",
  "gene": "UniProtKB:Q5VZP5",
  "term_id": "GO:0008138",
  "gene_symbol": "STYXL2"
}